{
  "gene_symbol": "HFE",
  "term_id": "GO:1990459",
  "gene_name": "Hereditary hemochromatosis protein",
  "gene": "UniProtKB:Q30201",
  "term_label": "transferrin receptor binding"
}